regulation of sprouting of injured axon [GO:0048686] (biological process) Relationships: is a type of GO:0022603; is_a regulation of developmental growth [GO:0048638]; is a type of regulation of extent of cell growth [GO:0061387]; regulates sprouting of injured axon [GO:0048682] Definition: Any process that modulates the frequency, rate or extent of sprouting of an injured axon. Sources: GOC:dgh, GOC:dph, GOC:jid, GOC:lm Subtypes: positive regulation of sprouting of injured axon [GO:0048687], negative regulation of sprouting of injured axon [GO:0048688], GO:0048690, GO:0048693, regulation of formation of growth cone in injured axon [GO:1905942]